{
  "gene": "UniProtKB:O95429",
  "term_id": "GO:0050821",
  "term_label": "protein stabilization",
  "gene_symbol": "BAG4",
  "gene_name": "BAG family molecular chaperone regulator 4"
}